{
  "term_label": "Unknown cellular component",
  "gene_name": "Peroxynitrite isomerase THAP4",
  "gene_symbol": "THAP4",
  "term_id": "UNKNOWN:0003",
  "gene": "UniProtKB:Q8WY91"
}